negative regulation of Hulle cell development [GO:0070809] (biological process) Definition: Any process that stops, prevents, or reduces the frequency, rate or extent of Hulle cell development, a process that leads to the formation of Hulle cells. Hulle cells are specialized multinucleate cells that originate from a nest-like aggregation of hyphae during sexual development and serve as nurse cells to the developing cleistothecium, or fruiting body. Relationships: is a type of negative regulation of cell development [GO:0010721]; is a type of regulation of Hulle cell development [GO:0070808]; is a type of negative regulation of reproductive process [GO:2000242]; negatively regulates GO:0070792 Sources: GOC:mah